{
  "term_label": "extracellular space",
  "gene_symbol": "NICOL1",
  "term_id": "GO:0005615",
  "gene": "UniProtKB:Q5BLP8",
  "gene_name": "Neuropeptide-like protein C4orf48"
}